{
  "gene_symbol": "TERF1",
  "term_id": "GO:1905839",
  "gene_name": "Telomeric repeat-binding factor 1",
  "term_label": "negative regulation of telomeric D-loop disassembly",
  "gene": "UniProtKB:P54274"
}